extrinsic component of plastid membrane [GO:0035452] (cellular component) Definition: The component of a plastid membrane consisting of gene products and protein complexes that are loosely bound to one of its surfaces, but not integrated into the hydrophobic region. Sources: GOC:bf, GOC:dos Also known as: peripheral to plastid membrane, extrinsic to plastid membrane Relationships: is a type of extrinsic component of organelle membrane [GO:0031312]; is part of plastid membrane [GO:0042170] Subtypes: extrinsic component of plastid thylakoid membrane [GO:0035449], extrinsic component of plastid inner membrane [GO:0035453]